{
  "term_id": "GO:0002430",
  "term_label": "complement receptor mediated signaling pathway",
  "gene": "UniProtKB:Q99788",
  "gene_symbol": "CMKLR1",
  "gene_name": "Chemerin-like receptor 1"
}